alpha-1,2-mannosyltransferase activity [GO:0000026] (MF) References: PMID:10521541 Sources: GOC:mcc Relationships: is a type of mannosyltransferase activity [GO:0000030] Subtypes: GDP-Man:Man(3)GlcNAc(2)-PP-Dol alpha-1,2-mannosyltransferase activity [GO:0004377], lipopolysaccharide N-acetylmannosaminouronosyltransferase activity [GO:0047241], dol-P-Man:Man(8)GlcNAc(2)-PP-Dol alpha-1,2-mannosyltransferase activity [GO:0052918], dol-P-Man:Man(6)GlcNAc(2)-PP-Dol alpha-1,2-mannosyltransferase activity [GO:0052926], GO:0120564, dol-P-Man:Man(3)GlcN-acyl-PI alpha-1,2-mannosyltransferase activity [GO:0120565] Definition: Catalysis of the transfer of a mannose residue to an oligosaccharide, forming an alpha-(1->2) linkage.